{
  "term_id": "GO:0009986",
  "gene": "UniProtKB:P18627",
  "gene_name": "Lymphocyte activation gene 3 protein",
  "gene_symbol": "LAG3",
  "term_label": "cell surface"
}